pancreatic amylase secretion [GO:0036395] (BP) Definition: The controlled release of amylase from a cell of the pancreas. References: PMID:19028687 Sources: GOC:jc Relationships: is a type of amylase secretion [GO:0036394]; is part of pancreatic juice secretion [GO:0030157] Regulation: regulated by regulation of pancreatic amylase secretion [GO:1902276]; negatively regulated by GO:1902277; positively regulated by positive regulation of pancreatic amylase secretion [GO:1902278]